{
  "gene": "UniProtKB:Q9NPI5",
  "gene_symbol": "NMRK2",
  "term_id": "GO:0005737",
  "term_label": "cytoplasm",
  "gene_name": "Nicotinamide riboside kinase 2"
}